{
  "term_id": "GO:0042073",
  "gene_name": "Intraflagellar transport protein 70B",
  "gene": "UniProtKB:Q8N4P2",
  "term_label": "intraciliary transport",
  "gene_symbol": "IFT70B"
}